regulation of response to G2 DNA damage checkpoint signaling [GO:1902157] (biological process) Definition: Any process that modulates the frequency, rate or extent of response to G2 DNA damage checkpoint signaling. Also known as: regulation of G2/M transition DNA damage checkpoint effector process, regulation of response to signal involved in G2/M transition DNA damage checkpoint Sources: GOC:TermGenie, GOC:mtg_cell_cycle Relationships: is a type of GO:1902153; regulates response to G2 DNA damage checkpoint signaling [GO:0072426] Subtypes: GO:1902158